regulation of development, heterochronic [GO:0040034] (biological process) References: PMID:9442909 Relationships: is a type of regulation of developmental process [GO:0050793] Subtypes: negative regulation of development, heterochronic [GO:0045961], GO:0045962, regulation of timing of animal organ formation [GO:0048504], regulation of timing of cell differentiation [GO:0048505], regulation of timing of meristematic phase transition [GO:0048506], GO:0090444, regulation of timing of plant organ formation [GO:0090709] Also known as: heterochronic regulation of development, temporal regulation of development, developmental timing Definition: Any process that modulates the consistent predetermined time point at which an integrated living unit or organism progresses from an initial condition to a later condition and the rate at which this time point is reached.